{
  "term_id": "UNKNOWN:0001",
  "gene_name": "Armadillo repeat-containing protein 8",
  "gene_symbol": "ARMC8",
  "term_label": "Unknown molecular function",
  "gene": "UniProtKB:Q8IUR7"
}